presynaptic endosome [GO:0098830] (cellular component) References: PMID:20200227, PMID:25939282 Relationships: is a type of endosome [GO:0005768]; is part of presynapse [GO:0098793] Note: As of 2015, there is still controversy over the nature of presynaptic endosomes and their relationship to regular endosomes. See Jahne et al., 2015 (PMID:25939282) for details. Definition: An endosome present in the presynapse that fuses with endocytic vesicles arising in the presynaptic endocytic zone. This organelle is believed to be involved in regeneration of synaptic vesicles.